{
  "gene_symbol": "CIROP",
  "gene": "UniProtKB:A0A1B0GTW7",
  "gene_name": "Ciliated left-right organizer metallopeptidase",
  "term_label": "peptidase activity",
  "term_id": "GO:0008233"
}